L-threonine transmembrane transporter activity [GO:0015195] (molecular function) Definition: Enables the transfer of L-threonine from one side of a membrane to the other. L-threonine is (2R*,3S*)-2-amino-3-hydroxybutanoic acid. Also known as: L-threonine transporter activity, L-threonine permease activity, threonine/serine:sodium symporter activity Subtypes: GO:0015565 Relationships: is a type of GO:0015175; is a type of L-amino acid transmembrane transporter activity [GO:0015179]; is part of threonine transport [GO:0015826] Sources: GOC:ai, GOC:mtg_transport, ISBN:0815340729